{
  "gene_name": "Dynamin-like 120 kDa protein, mitochondrial",
  "gene_symbol": "OPA1",
  "gene": "UniProtKB:O60313",
  "term_label": "mitochondrial membrane",
  "term_id": "GO:0031966"
}